{
  "term_label": "nucleus",
  "gene_name": "Histone H2B type 3-B",
  "term_id": "GO:0005634",
  "gene": "UniProtKB:Q8N257",
  "gene_symbol": "H2BC26"
}